{
  "term_id": "GO:0001665",
  "term_label": "alpha-N-acetylgalactosaminide alpha-2,6-sialyltransferase activity",
  "gene": "UniProtKB:Q969X2",
  "gene_name": "Alpha-N-acetylgalactosaminide alpha-2,6-sialyltransferase 6",
  "gene_symbol": "ST6GALNAC6"
}